dense core granule priming [GO:0061789] (biological process) References: PMID:10899113, PMID:26575293 Sources: GOC:PARL, GOC:bf Definition: A process that converts unprimed dense core granules (DCVs) to a pool of primed vesicles that are capable of fusing with the plasma membrane (fusion-competent) and thereby releasing their contents. Priming typically occurs after docking. Also known as: LDCV priming, dense core vesicle priming, large dense-core vesicle priming Relationships: is_a protein-containing complex assembly [GO:0065003]; is a type of exocytic process [GO:0140029]; is part of dense core granule exocytosis [GO:1990504]